thyrotropin-releasing hormone receptor binding [GO:0031531] (MF) Relationships: is a type of G protein-coupled receptor binding [GO:0001664]; is a type of peptide hormone receptor binding [GO:0051428] Also known as: thyrotropin releasing hormone receptor binding, thyrotropin-releasing hormone receptor ligand References: PMID:8592728 Definition: Binding to a receptor for thyrotropin-releasing hormone, a tripeptide hormone that is produced by the hypothalamus and stimulates the release of thyroid-stimulating hormone (TSH) and prolactin by the anterior pituitary.